fucose catabolic process [GO:0019317] (biological process) Definition: The chemical reactions and pathways resulting in the breakdown of fucose (6-deoxygalactose). Also known as: fucose breakdown, fucose catabolism, fucose degradation Relationships: is a type of fucose metabolic process [GO:0006004]; is a type of hexose catabolic process [GO:0019320] Subtypes: GO:0042355 Regulation: regulated by regulation of fucose catabolic process [GO:0043468] Sources: GOC:jl